{
  "term_id": "UNKNOWN:0001",
  "gene": "UniProtKB:A0A804HI29",
  "gene_symbol": "A0A804HI29",
  "gene_name": "Uncharacterized protein",
  "term_label": "Unknown molecular function"
}